{
  "gene_symbol": "ZNF219",
  "term_label": "RNA polymerase II cis-regulatory region sequence-specific DNA binding",
  "gene": "UniProtKB:Q9P2Y4",
  "gene_name": "Zinc finger protein 219",
  "term_id": "GO:0000978"
}